{
  "gene": "UniProtKB:P28329",
  "term_id": "GO:0007274",
  "gene_name": "Choline O-acetyltransferase",
  "gene_symbol": "CHAT",
  "term_label": "neuromuscular synaptic transmission"
}